{
  "term_label": "cytosol",
  "gene_name": "Ubiquitin carboxyl-terminal hydrolase 46",
  "gene_symbol": "USP46",
  "gene": "UniProtKB:P62068",
  "term_id": "GO:0005829"
}